{
  "gene_name": "Olfactory receptor 2A12",
  "term_id": "GO:0050911",
  "term_label": "detection of chemical stimulus involved in sensory perception of smell",
  "gene_symbol": "OR2A12",
  "gene": "UniProtKB:Q8NGT7"
}